{
  "gene": "UniProtKB:Q14493",
  "gene_name": "Histone RNA hairpin-binding protein",
  "term_label": "cytoplasm",
  "gene_symbol": "SLBP",
  "term_id": "GO:0005737"
}